fat cell differentiation [GO:0045444] (BP) Definition: The process in which a relatively unspecialized cell acquires specialized features of an adipocyte, an animal connective tissue cell specialized for the synthesis and storage of fat. Sources: CL:0000136, GOC:go_curators Regulation: regulated by regulation of fat cell differentiation [GO:0045598]; negatively regulated by negative regulation of fat cell differentiation [GO:0045599]; positively regulated by GO:0045600 Subtypes: white fat cell differentiation [GO:0050872], GO:0050873, GO:0160274 Also known as: adipocyte cell differentiation, adipocyte differentiation, adipose cell differentiation, adipogenesis Relationships: is_a GO:0030154